{
  "gene_name": "Microphthalmia-associated transcription factor",
  "term_label": "nucleus",
  "gene": "UniProtKB:O75030",
  "gene_symbol": "MITF",
  "term_id": "GO:0005634"
}